{
  "term_id": "GO:0003823",
  "gene_name": "Immunoglobulin heavy variable 1-18",
  "gene_symbol": "IGHV1-18",
  "term_label": "antigen binding",
  "gene": "UniProtKB:A0A0C4DH31"
}